{
  "gene_symbol": "DCLRE1C",
  "term_id": "GO:0036297",
  "term_label": "interstrand cross-link repair",
  "gene_name": "Protein artemis",
  "gene": "UniProtKB:Q96SD1"
}